{
  "gene": "UniProtKB:Q5SRH9",
  "term_id": "UNKNOWN:0002",
  "gene_symbol": "TTC39A",
  "term_label": "Unknown biological process",
  "gene_name": "Tetratricopeptide repeat protein 39A"
}